{
  "gene_symbol": "CTTN",
  "gene_name": "Src substrate cortactin",
  "gene": "UniProtKB:Q14247",
  "term_label": "endocytic vesicle",
  "term_id": "GO:0030139"
}